{
  "gene_symbol": "ARHGEF3",
  "term_id": "GO:0035025",
  "gene": "UniProtKB:Q9NR81",
  "gene_name": "Rho guanine nucleotide exchange factor 3",
  "term_label": "positive regulation of Rho protein signal transduction"
}